{
  "gene_name": "AF4_FMR2 family member 2",
  "gene": "UniProtKB:P51816",
  "gene_symbol": "AFF2",
  "term_id": "GO:0006355",
  "term_label": "regulation of DNA-templated transcription"
}